{
  "gene": "UniProtKB:Q9GZM7",
  "gene_name": "Tubulointerstitial nephritis antigen-like",
  "term_label": "Unknown biological process",
  "term_id": "UNKNOWN:0002",
  "gene_symbol": "TINAGL1"
}